{
  "gene_symbol": "FASTKD5",
  "term_label": "regulation of mitochondrial mRNA stability",
  "gene": "UniProtKB:Q7L8L6",
  "gene_name": "FAST kinase domain-containing protein 5, mitochondrial",
  "term_id": "GO:0044528"
}